ribonucleotide excision repair [GO:1990516] (biological process) Relationships: is a type of mismatch repair involved in maintenance of fidelity involved in DNA-dependent DNA replication [GO:0070716] Definition: The pathway by which a ribonucleotide is removed from DNA and replaced by a deoxyribonucleotide. The ribonucleotide is incised by RNase H2, and further excised by an endonuclease. The resulting 1 nt gap is then repaired by DNA polymerase and DNA ligase. References: PMID:12475934, PMID:22864116